{
  "gene_name": "Putative uncharacterized protein DHRS4-AS1",
  "term_label": "Unknown cellular component",
  "gene": "UniProtKB:Q9P1J3",
  "gene_symbol": "DHRS4-AS1",
  "term_id": "UNKNOWN:0003"
}